{
  "gene_symbol": "HSD17B8",
  "gene_name": "(3R)-3-hydroxyacyl-CoA dehydrogenase",
  "gene": "UniProtKB:Q92506",
  "term_label": "quinone binding",
  "term_id": "GO:0048038"
}